{
  "term_label": "regulation of canonical Wnt signaling pathway",
  "term_id": "GO:0060828",
  "gene_name": "Serine_threonine-protein phosphatase 2A regulatory subunit B'' subunit alpha",
  "gene_symbol": "PPP2R3A",
  "gene": "UniProtKB:Q06190"
}